{
  "gene": "UniProtKB:O95258",
  "gene_symbol": "SLC25A14",
  "term_id": "GO:0015078",
  "gene_name": "Brain mitochondrial carrier protein 1",
  "term_label": "proton transmembrane transporter activity"
}